{
  "gene_symbol": "RBCK1",
  "gene": "UniProtKB:Q9BYM8",
  "term_id": "GO:0043130",
  "gene_name": "RanBP-type and C3HC4-type zinc finger-containing protein 1",
  "term_label": "ubiquitin binding"
}